phosphatidylethanolamine floppase activity [GO:0140341] (molecular function) Definition: Catalysis of the movement of phosphatidylethanolamine from the cytosolic to the exoplasmic leaflet of a membrane, using energy from the hydrolysis of ATP. Relationships: is a type of phospholipid transporter activity [GO:0005548]; is a type of floppase activity [GO:0140328] References: PMID:10029989 Also known as: phosphatidylethanolamine floppase activity (cytosolic to exoplasmic leaflet)